{
  "gene_name": "Zinc finger protein 682",
  "gene": "UniProtKB:O95780",
  "term_id": "GO:0006355",
  "term_label": "regulation of DNA-templated transcription",
  "gene_symbol": "ZNF682"
}